{
  "gene_symbol": "MRPL42",
  "gene_name": "Large ribosomal subunit protein mL42",
  "term_id": "UNKNOWN:0002",
  "term_label": "Unknown biological process",
  "gene": "UniProtKB:Q9Y6G3"
}